pyridoxine 5'-O-beta-D-glucosyltransferase activity [GO:0047231] (MF) Definition: Catalysis of the reaction: pyridoxine + UDP-D-glucose = 5'-O-beta-D-glucosylpyridoxine + H+ + UDP. Sources: EC:2.4.1.160, RHEA:20177 Also known as: UDP-glucose-pyridoxine glucosyltransferase activity, UDP-glucose:pyridoxine 5'-O-beta-D-glucosyltransferase activity, UDP-glucose:pyridoxine 5'-O-beta-glucosyltransferase activity, UDPglucose:pyridoxine 5'-O-beta-D-glucosyltransferase activity, uridine diphosphoglucose-pyridoxine 5'-beta-glucosyltransferase activity Relationships: is_a GO:0035251